{
  "gene_symbol": "H2BC11",
  "term_label": "extracellular space",
  "gene_name": "Histone H2B type 1-J",
  "term_id": "GO:0005615",
  "gene": "UniProtKB:P06899"
}